{
  "term_label": "RISC-loading complex",
  "gene_symbol": "DICER1",
  "gene": "UniProtKB:Q9UPY3",
  "term_id": "GO:0070578",
  "gene_name": "Endoribonuclease Dicer"
}